{
  "term_label": "Unknown molecular function",
  "gene_name": "Transmembrane protein 109",
  "gene_symbol": "TMEM109",
  "term_id": "UNKNOWN:0001",
  "gene": "UniProtKB:Q9BVC6"
}